{
  "term_id": "UNKNOWN:0003",
  "term_label": "Unknown cellular component",
  "gene_name": "Leukocyte receptor cluster member 9",
  "gene": "UniProtKB:Q96B70",
  "gene_symbol": "LENG9"
}